{
  "gene_name": "Zinc finger protein 773",
  "gene_symbol": "ZNF773",
  "term_label": "regulation of transcription by RNA polymerase II",
  "gene": "UniProtKB:Q6PK81",
  "term_id": "GO:0006357"
}